{
  "term_id": "UNKNOWN:0001",
  "gene": "UniProtKB:Q9BZL3",
  "term_label": "Unknown molecular function",
  "gene_name": "Small integral membrane protein 3",
  "gene_symbol": "SMIM3"
}